{
  "gene": "UniProtKB:Q9BTW9",
  "term_id": "GO:0016328",
  "gene_symbol": "TBCD",
  "term_label": "lateral plasma membrane",
  "gene_name": "Tubulin-specific chaperone D"
}